{
  "gene_name": "Glucose-6-phosphate exchanger SLC37A2",
  "term_label": "glucose 6-phosphate:phosphate antiporter activity",
  "term_id": "GO:0061513",
  "gene_symbol": "SLC37A2",
  "gene": "UniProtKB:Q8TED4"
}